{
  "gene_symbol": "KRT32",
  "term_label": "structural constituent of skin epidermis",
  "gene": "UniProtKB:Q14532",
  "term_id": "GO:0030280",
  "gene_name": "Keratin, type I cuticular Ha2"
}